{
  "term_label": "Unknown molecular function",
  "term_id": "UNKNOWN:0001",
  "gene_name": "Vesicle-trafficking protein SEC22c",
  "gene_symbol": "SEC22C",
  "gene": "UniProtKB:Q9BRL7"
}